{
  "term_id": "GO:0070721",
  "term_label": "ISGF3 complex",
  "gene": "UniProtKB:P52630",
  "gene_name": "Signal transducer and activator of transcription 2",
  "gene_symbol": "STAT2"
}